{
  "gene": "UniProtKB:Q9BYD9",
  "term_id": "GO:0015629",
  "term_label": "actin cytoskeleton",
  "gene_symbol": "ACTRT3",
  "gene_name": "Actin-related protein T3"
}